{
  "term_label": "cilium",
  "gene": "UniProtKB:Q99835",
  "gene_name": "Protein smoothened",
  "term_id": "GO:0005929",
  "gene_symbol": "SMO"
}